poly(hydroxyalkanoate) biosynthetic process [GO:1901441] (biological process) Relationships: is a type of biosynthetic process [GO:0009058]; is a type of poly(hydroxyalkanoate) metabolic process [GO:1901440] Also known as: poly(hydroxyalkanoate) anabolism, poly(hydroxyalkanoate) biosynthesis, poly(hydroxyalkanoate) formation, poly(hydroxyalkanoate) synthesis Subtypes: poly-hydroxybutyrate biosynthetic process [GO:0042619], GO:1902921, poly(hydroxyalkanoate) biosynthetic process from glucose [GO:1902924], poly(hydroxyalkanoate) biosynthetic process from fatty acid [GO:1902925] Definition: The chemical reactions and pathways resulting in the formation of poly(hydroxyalkanoate). Sources: GOC:TermGenie, GOC:mengo_curators